vulval development [GO:0040025] (biological process) Definition: The process whose specific outcome is the progression of the egg-laying organ of female and hermaphrodite nematodes over time, from its formation to the mature structure. In nematodes, the vulva is formed from ventral epidermal cells during larval stages to give rise to a fully formed vulva in the adult. Regulation: positively regulated by positive regulation of vulval development [GO:0040026]; negatively regulated by negative regulation of vulval development [GO:0040027]; regulated by regulation of vulval development [GO:0040028] Sources: GOC:ems, GOC:kmv, ISBN:087969307X Relationships: is a type of animal organ development [GO:0048513]; is part of nematode larval development [GO:0002119]